{
  "gene_symbol": "SPAG6",
  "gene": "UniProtKB:O75602",
  "gene_name": "Sperm-associated antigen 6",
  "term_id": "GO:0005930",
  "term_label": "axoneme"
}